{
  "term_label": "immune response",
  "gene_symbol": "LAT",
  "gene": "UniProtKB:O43561",
  "term_id": "GO:0006955",
  "gene_name": "Linker for activation of T-cells family member 1"
}